{
  "term_label": "positive regulation of axonogenesis",
  "gene": "UniProtKB:Q9H9P2",
  "gene_name": "Chondrolectin",
  "gene_symbol": "CHODL",
  "term_id": "GO:0050772"
}